negative regulation of dCDP biosynthetic process [GO:1903529] (biological process) Also known as: down regulation of dCDP anabolism, down regulation of dCDP biosynthesis, down regulation of dCDP biosynthetic process, down regulation of dCDP formation, down regulation of dCDP synthesis, down-regulation of dCDP anabolism, down-regulation of dCDP biosynthesis, down-regulation of dCDP biosynthetic process, down-regulation of dCDP formation, down-regulation of dCDP synthesis, downregulation of dCDP anabolism, downregulation of dCDP biosynthesis, downregulation of dCDP biosynthetic process, downregulation of dCDP formation, downregulation of dCDP synthesis, negative regulation of dCDP anabolism, negative regulation of dCDP biosynthesis, negative regulation of dCDP formation, negative regulation of dCDP synthesis, inhibition of dCDP anabolism, inhibition of dCDP biosynthesis, inhibition of dCDP biosynthetic process, inhibition of dCDP formation, inhibition of dCDP synthesis Definition: Any process that stops, prevents or reduces the frequency, rate or extent of dCDP biosynthetic process. References: PMID:16317005 Sources: GOC:TermGenie, GO_REF:0000058 Relationships: is a type of negative regulation of pyrimidine nucleotide biosynthetic process [GO:1900398]; is a type of regulation of dCDP biosynthetic process [GO:1903528]; negatively regulates dCDP biosynthetic process [GO:0006240]